negative regulation of leukocyte mediated cytotoxicity [GO:0001911] (biological process) References: PMID:11911826 Sources: GOC:add, ISBN:0781735149 Relationships: is a type of regulation of leukocyte mediated cytotoxicity [GO:0001910]; is a type of GO:0002704; is a type of negative regulation of cell killing [GO:0031342]; negatively regulates leukocyte mediated cytotoxicity [GO:0001909] Subtypes: GO:0001814, negative regulation of T cell mediated cytotoxicity [GO:0001915], negative regulation of natural killer cell mediated cytotoxicity [GO:0045953], GO:0070954, GO:1904150 Also known as: down regulation of leukocyte mediated cytotoxicity, down-regulation of leukocyte mediated cytotoxicity, downregulation of leukocyte mediated cytotoxicity, negative regulation of immune cell mediated cytotoxicity, negative regulation of leucocyte mediated cytotoxicity, inhibition of leukocyte mediated cytotoxicity Definition: Any process that stops, prevents, or reduces the rate of leukocyte mediated cytotoxicity.